{
  "gene_symbol": "SKOR2",
  "term_id": "GO:0005634",
  "gene": "UniProtKB:Q2VWA4",
  "gene_name": "SKI family transcriptional corepressor 2",
  "term_label": "nucleus"
}